3D-(3,5/4)-trihydroxycyclohexane-1,2-dione hydrolase activity [GO:0102481] (molecular function) Definition: Catalysis of the reaction: 3D-3,5/4-trihydroxycyclohexane-1,2-dione + H2O = 5-deoxy-D-glucuronate + H+. Sources: GOC:pz, RHEA:25836 Relationships: is a type of hydrolase activity, acting on acid carbon-carbon bonds, in ketonic substances [GO:0016823]